{
  "gene": "UniProtKB:Q15345",
  "gene_name": "Leucine-rich repeat-containing protein 41",
  "term_id": "GO:0005634",
  "term_label": "nucleus",
  "gene_symbol": "LRRC41"
}